alpha,alpha-phosphotrehalase activity [GO:0008788] (molecular function) Relationships: is a type of trehalase activity [GO:0015927] Also known as: alpha,alpha-trehalose-6-phosphate phosphoglucohydrolase activity, phosphotrehalase activity, trehalose-6-phosphate hydrolase activity Definition: Catalysis of the reaction: alpha,alpha-trehalose 6-phosphate + H2O = D-glucose + D-glucose 6-phosphate. Sources: EC:3.2.1.93